quinaldate 4-oxidoreductase activity [GO:0047122] (molecular function) Sources: EC:1.3.99.18, RHEA:16697 Also known as: quinaldic acid 4-oxidoreductase activity, quinoline-2-carboxylate:acceptor 4-oxidoreductase (hydroxylating) Definition: Catalysis of the reaction: A + H2O + quinaldate = AH(2) + kynurenate. Relationships: is a type of oxidoreductase activity, acting on the CH-CH group of donors [GO:0016627]